{
  "term_id": "GO:0005634",
  "gene_symbol": "PHF12",
  "gene": "UniProtKB:Q96QT6",
  "term_label": "nucleus",
  "gene_name": "PHD finger protein 12"
}